{
  "term_id": "UNKNOWN:0001",
  "term_label": "Unknown molecular function",
  "gene_name": "C1GALT1-specific chaperone 1-like protein",
  "gene_symbol": "C1GALT1C1L",
  "gene": "UniProtKB:P0DN25"
}